{
  "gene": "UniProtKB:Q6EEV6",
  "term_label": "protein tag activity",
  "term_id": "GO:0031386",
  "gene_symbol": "SUMO4",
  "gene_name": "Small ubiquitin-related modifier 4"
}